anaphase-promoting complex binding [GO:0010997] (molecular function) Definition: Binding to an anaphase-promoting complex. A ubiquitin ligase complex that degrades mitotic cyclins and anaphase inhibitory protein, thereby triggering sister chromatid separation and exit from mitosis. Also known as: APC binding Relationships: is_a protein-containing complex binding [GO:0044877] Sources: GOC:BHF, GOC:dph, GOC:tb